{
  "term_id": "GO:0019722",
  "gene_name": "Sterile alpha motif domain-containing protein 14",
  "term_label": "calcium-mediated signaling",
  "gene": "UniProtKB:Q8IZD0",
  "gene_symbol": "SAMD14"
}